{
  "gene_name": "WD repeat-containing protein 54",
  "term_label": "Unknown biological process",
  "gene": "UniProtKB:Q9H977",
  "gene_symbol": "WDR54",
  "term_id": "UNKNOWN:0002"
}